{
  "term_label": "ubiquitin-like ligase-substrate adaptor activity",
  "term_id": "GO:1990756",
  "gene": "UniProtKB:Q96JP0",
  "gene_symbol": "FEM1C",
  "gene_name": "Protein fem-1 homolog C"
}